{
  "gene": "UniProtKB:Q9UPQ9",
  "gene_name": "Trinucleotide repeat-containing gene 6B protein",
  "term_label": "positive regulation of nuclear-transcribed mRNA poly(A) tail shortening",
  "gene_symbol": "TNRC6B",
  "term_id": "GO:0060213"
}